{
  "gene_name": "MOB kinase activator 1B",
  "gene": "UniProtKB:Q7L9L4",
  "gene_symbol": "MOB1B",
  "term_label": "nucleus",
  "term_id": "GO:0005634"
}